serotonin-gated chloride channel activity [GO:0160039] (MF) Relationships: is_a GO:0005254; is_a transmitter-gated monoatomic ion channel activity [GO:0022824]; is a type of ligand-gated monoatomic anion channel activity [GO:0099095]; is a type of GO:0099589; is part of serotonin receptor signaling pathway [GO:0007210] References: PMID:11100728 Definition: Enables the transmembrane transfer of a chloride ion by a channel that opens when the biogenic amine serotonin has been bound by the channel complex or one of its constituent parts. Serotonin (5-hydroxytryptamine) is a neurotransmitter and hormone found in vertebrates and invertebrates.